{
  "gene_symbol": "FADS6",
  "gene_name": "Fatty acid desaturase 6",
  "gene": "UniProtKB:Q8N9I5",
  "term_id": "GO:0016020",
  "term_label": "membrane"
}